G protein-coupled receptor signaling pathway involved in defense response to Gram-negative bacterium [GO:1903554] (biological process) Also known as: G protein coupled receptor protein signaling pathway involved in defence response to Gram-negative bacteria, G protein coupled receptor protein signaling pathway involved in defence response to Gram-negative bacterium, G protein coupled receptor protein signaling pathway involved in defense response to Gram-negative bacteria, G protein coupled receptor protein signaling pathway involved in defense response to Gram-negative bacterium, G protein coupled receptor protein signalling pathway involved in defence response to Gram-negative bacteria, G protein coupled receptor protein signalling pathway involved in defence response to Gram-negative bacterium, G protein coupled receptor protein signalling pathway involved in defense response to Gram-negative bacteria, G protein coupled receptor protein signalling pathway involved in defense response to Gram-negative bacterium, G-protein coupled receptor protein signal transduction involved in defence response to Gram-negative bacteria, G-protein coupled receptor protein signal transduction involved in defence response to Gram-negative bacterium, G-protein coupled receptor protein signal transduction involved in defense response to Gram-negative bacteria, G-protein coupled receptor protein signal transduction involved in defense response to Gram-negative bacterium, G-protein coupled receptor protein signaling pathway involved in defence response to Gram-negative bacteria, G-protein coupled receptor protein signaling pathway involved in defence response to Gram-negative bacterium, G-protein coupled receptor protein signaling pathway involved in defense response to Gram-negative bacteria, G-protein coupled receptor protein signaling pathway involved in defense response to Gram-negative bacterium, G-protein coupled receptor signaling pathway involved in defence response to Gram-negative bacteria, G-protein coupled receptor signaling pathway involved in defence response to Gram-negative bacterium, G-protein coupled receptor signaling pathway involved in defense response to Gram-negative bacteria, G-protein coupled receptor signalling pathway involved in defence response to Gram-negative bacteria, G-protein coupled receptor signalling pathway involved in defence response to Gram-negative bacterium, G-protein coupled receptor signalling pathway involved in defense response to Gram-negative bacteria, G-protein coupled receptor signalling pathway involved in defense response to Gram-negative bacterium, G-protein-coupled receptor protein signaling pathway involved in defence response to Gram-negative bacteria, G-protein-coupled receptor protein signaling pathway involved in defence response to Gram-negative bacterium, G-protein-coupled receptor protein signaling pathway involved in defense response to Gram-negative bacterium, G-protein-coupled receptor protein signalling pathway involved in defence response to Gram-negative bacteria, G-protein-coupled receptor protein signalling pathway involved in defence response to Gram-negative bacterium, G-protein-coupled receptor protein signalling pathway involved in defense response to Gram-negative bacteria, G-protein-coupled receptor protein signalling pathway involved in defense response to Gram-negative bacterium, GPCR signaling pathway involved in defence response to Gram-negative bacteria, GPCR signaling pathway involved in defence response to Gram-negative bacterium, GPCR signaling pathway involved in defense response to Gram-negative bacteria, GPCR signaling pathway involved in defense response to Gram-negative bacterium, GPCR signalling pathway involved in defence response to Gram-negative bacteria, GPCR signalling pathway involved in defence response to Gram-negative bacterium, GPCR signalling pathway involved in defense response to Gram-negative bacteria, GPCR signalling pathway involved in defense response to Gram-negative bacterium, G protein coupled receptor protein signaling pathway involved in Gram-negative antibacterial peptide activity, G protein coupled receptor protein signalling pathway involved in Gram-negative antibacterial peptide activity, G-protein coupled receptor protein signal transduction involved in Gram-negative antibacterial peptide activity, G-protein coupled receptor protein signaling pathway involved in Gram-negative antibacterial peptide activity, G-protein coupled receptor signaling pathway involved in Gram-negative antibacterial peptide activity, G-protein coupled receptor signalling pathway involved in Gram-negative antibacterial peptide activity, G-protein-coupled receptor protein signaling pathway involved in Gram-negative antibacterial peptide activity, G-protein-coupled receptor protein signalling pathway involved in Gram-negative antibacterial peptide activity, GPCR signaling pathway involved in Gram-negative antibacterial peptide activity, GPCR signalling pathway involved in Gram-negative antibacterial peptide activity References: PMID:25303524 Sources: GOC:TermGenie, GOC:kmv, GO_REF:0000060 Definition: A G protein-coupled receptor signaling pathway that is involved in the defense response to Gram-negative bacterium. Relationships: is a type of G protein-coupled receptor signaling pathway [GO:0007186]; BFO_0000050 defense response to Gram-negative bacterium [GO:0050829]